{
  "term_id": "UNKNOWN:0001",
  "gene_name": "Mitotic spindle assembly checkpoint protein MAD1",
  "gene_symbol": "MAD1L1",
  "gene": "UniProtKB:Q9Y6D9",
  "term_label": "Unknown molecular function"
}